early endosome [GO:0005769] (CC) References: PMID:19696797 Sources: GOC:mah, NIF_Subcellular:nlx_subcell_20090701 Subtypes: postsynaptic early endosome [GO:0098842] Definition: A membrane-bounded organelle that receives incoming material from primary endocytic vesicles that have been generated by clathrin-dependent and clathrin-independent endocytosis; vesicles fuse with the early endosome to deliver cargo for sorting into recycling or degradation pathways. Relationships: is a type of endosome [GO:0005768]